{
  "gene_symbol": "ACAD9",
  "gene": "UniProtKB:Q9H845",
  "gene_name": "Complex I assembly factor ACAD9, mitochondrial",
  "term_label": "Unknown cellular component",
  "term_id": "UNKNOWN:0003"
}